{
  "term_label": "centrosome",
  "term_id": "GO:0005813",
  "gene_name": "Centrosomal protein of 44 kDa",
  "gene_symbol": "CEP44",
  "gene": "UniProtKB:Q9C0F1"
}